{
  "gene": "UniProtKB:O43307",
  "gene_name": "Rho guanine nucleotide exchange factor 9",
  "term_id": "GO:0005829",
  "gene_symbol": "ARHGEF9",
  "term_label": "cytosol"
}